SUMO activating enzyme complex [GO:0031510] (cellular component) Definition: A conserved heterodimeric complex with SUMO activating enzyme activity. References: PMID:15601841 Also known as: SAE, SUMO E1 activator enzyme complex Relationships: is a type of nuclear protein-containing complex [GO:0140513]; is a type of catalytic complex [GO:1902494]